{
  "term_id": "GO:0006888",
  "gene_name": "General vesicular transport factor p115",
  "gene_symbol": "USO1",
  "gene": "UniProtKB:O60763",
  "term_label": "endoplasmic reticulum to Golgi vesicle-mediated transport"
}